negative regulation of beta-catenin-TCF complex assembly [GO:1904864] (biological process) Relationships: is a type of negative regulation of protein-containing complex assembly [GO:0031333]; is a type of regulation of beta-catenin-TCF complex assembly [GO:1904863]; negatively regulates beta-catenin-TCF complex assembly [GO:1904837] References: PMID:18936100 Sources: GOC:PARL, GOC:TermGenie, GOC:bf, GO_REF:0000058 Also known as: down regulation of beta-catenin-TCF complex assembly, down regulation of beta-catenin-TCF complex formation, down-regulation of beta-catenin-TCF complex assembly, down-regulation of beta-catenin-TCF complex formation, downregulation of beta-catenin-TCF complex assembly, downregulation of beta-catenin-TCF complex formation, negative regulation of beta-catenin-TCF complex formation, down regulation of beta-catenin/LEF complex assembly, down regulation of beta-catenin/LEF complex formation, down-regulation of beta-catenin/LEF complex assembly, down-regulation of beta-catenin/LEF complex formation, downregulation of beta-catenin/LEF complex assembly, downregulation of beta-catenin/LEF complex formation, inhibition of beta-catenin-TCF complex assembly, inhibition of beta-catenin-TCF complex formation, inhibition of beta-catenin/LEF complex assembly, inhibition of beta-catenin/LEF complex formation, negative regulation of beta-catenin/LEF complex assembly, negative regulation of beta-catenin/LEF complex formation, down regulation of beta-catenin/T-cell factor complex assembly, down regulation of beta-catenin/T-cell factor complex formation, down regulation of beta-catenin/lymphoid enhancer binding factor complex assembly, down regulation of beta-catenin/lymphoid enhancer binding factor complex formation, down-regulation of beta-catenin/T-cell factor complex assembly, down-regulation of beta-catenin/T-cell factor complex formation, down-regulation of beta-catenin/lymphoid enhancer binding factor complex assembly, down-regulation of beta-catenin/lymphoid enhancer binding factor complex formation, downregulation of beta-catenin/T-cell factor complex assembly, downregulation of beta-catenin/T-cell factor complex formation, downregulation of beta-catenin/lymphoid enhancer binding factor complex assembly, downregulation of beta-catenin/lymphoid enhancer binding factor complex formation, inhibition of beta-catenin/T-cell factor complex assembly, inhibition of beta-catenin/T-cell factor complex formation, inhibition of beta-catenin/lymphoid enhancer binding factor complex assembly, inhibition of beta-catenin/lymphoid enhancer binding factor complex formation, negative regulation of beta-catenin/T-cell factor complex assembly, negative regulation of beta-catenin/T-cell factor complex formation, negative regulation of beta-catenin/lymphoid enhancer binding factor complex assembly, negative regulation of beta-catenin/lymphoid enhancer binding factor complex formation Definition: Any process that stops, prevents or reduces the frequency, rate or extent of beta-catenin-TCF complex assembly.